{
  "gene_name": "Probable ATP-dependent RNA helicase DDX46",
  "gene": "UniProtKB:Q7L014",
  "gene_symbol": "DDX46",
  "term_id": "GO:0005634",
  "term_label": "nucleus"
}